{
  "term_id": "GO:0098794",
  "gene_name": "Gamma-aminobutyric acid receptor subunit alpha-5",
  "term_label": "postsynapse",
  "gene": "UniProtKB:P31644",
  "gene_symbol": "GABRA5"
}